{
  "term_label": "chitin catabolic process",
  "gene_symbol": "CHI3L2",
  "gene": "UniProtKB:Q15782",
  "term_id": "GO:0006032",
  "gene_name": "Chitinase-3-like protein 2"
}